positive regulation of dendritic cell antigen processing and presentation [GO:0002606] (biological process) Definition: Any process that activates or increases the frequency, rate, or extent of dendritic cell antigen processing and presentation. Subtypes: positive regulation of myeloid dendritic cell antigen processing and presentation [GO:0002609], positive regulation of plasmacytoid dendritic cell antigen processing and presentation [GO:0002612] Sources: GOC:add Also known as: up regulation of dendritic cell antigen processing and presentation, up-regulation of dendritic cell antigen processing and presentation, upregulation of dendritic cell antigen processing and presentation, activation of dendritic cell antigen processing and presentation, stimulation of dendritic cell antigen processing and presentation Relationships: is a type of positive regulation of antigen processing and presentation [GO:0002579]; is a type of regulation of dendritic cell antigen processing and presentation [GO:0002604]; positively regulates dendritic cell antigen processing and presentation [GO:0002468]